{
  "term_id": "GO:0004386",
  "gene_name": "ATP-dependent RNA helicase DQX1",
  "term_label": "helicase activity",
  "gene": "UniProtKB:Q8TE96",
  "gene_symbol": "DQX1"
}